{
  "term_label": "negative regulation of gene expression via chromosomal CpG island methylation",
  "gene_symbol": "DNMT1",
  "term_id": "GO:0044027",
  "gene_name": "DNA (cytosine-5)-methyltransferase 1",
  "gene": "UniProtKB:P26358"
}